{
  "gene_name": "Thioredoxin domain-containing protein 3",
  "term_label": "flagellated sperm motility",
  "gene": "UniProtKB:Q8N427",
  "term_id": "GO:0030317",
  "gene_symbol": "NME8"
}